{
  "gene": "UniProtKB:Q8N257",
  "term_id": "GO:0019731",
  "term_label": "antibacterial humoral response",
  "gene_symbol": "H2BC26",
  "gene_name": "Histone H2B type 3-B"
}